tRNA (adenine) methyltransferase activity [GO:0016426] (molecular function) Subtypes: tRNA (adenine(37)-C2)-methyltransferase activity [GO:0002935], tRNA (adenine-N6)-methyltransferase activity [GO:0016430], tRNA (adenine(57)-N1)/(adenine(58)-N1)-methyltransferase activity [GO:0043827], tRNA (L-threonylcarbamoyladenosine(37)-C2) methyltransferase activity [GO:0089715], GO:0160105, tRNA (adenine(9)-N1)-methyltransferase activity [GO:0160106], tRNA (adenine(58)-N1)-methyltransferase activity [GO:0160107] Sources: GOC:go-curators Also known as: tRNA (adenine-C2-)-methyltransferase activity Definition: Catalysis of the reaction: S-adenosyl-L-methionine + tRNA = S-adenosyl-L-homocysteine + tRNA containing methyladenine. Relationships: is a type of tRNA methyltransferase activity [GO:0008175]; is a type of S-adenosylmethionine-dependent methyltransferase activity [GO:0008757]